{
  "gene_name": "Golgi-associated RAB2 interactor protein 5A",
  "term_id": "UNKNOWN:0001",
  "gene": "UniProtKB:Q6IPT2",
  "gene_symbol": "GARIN5A",
  "term_label": "Unknown molecular function"
}